{
  "gene": "UniProtKB:Q99963",
  "gene_name": "Endophilin-A3",
  "gene_symbol": "SH3GL3",
  "term_label": "glutamatergic synapse",
  "term_id": "GO:0098978"
}